extracellular matrix assembly [GO:0085029] (biological process) Sources: GOC:jl Regulation: regulated by regulation of extracellular matrix assembly [GO:1901201]; negatively regulated by negative regulation of extracellular matrix assembly [GO:1901202]; positively regulated by positive regulation of extracellular matrix assembly [GO:1901203] Relationships: is a type of cellular component assembly [GO:0022607]; is a type of extracellular matrix organization [GO:0030198] Definition: The aggregation, arrangement and bonding together of the extracellular matrix. Subtypes: vitelline membrane formation [GO:0030704], elastic fiber assembly [GO:0048251], GO:0070831, biofilm matrix assembly [GO:0098785]